{
  "gene": "UniProtKB:A5D8T8",
  "gene_name": "C-type lectin domain family 18 member A",
  "term_id": "GO:0030247",
  "term_label": "polysaccharide binding",
  "gene_symbol": "CLEC18A"
}